{
  "term_label": "Unknown molecular function",
  "term_id": "UNKNOWN:0001",
  "gene": "UniProtKB:A0A075B6N3",
  "gene_name": "T cell receptor beta variable 24-1",
  "gene_symbol": "TRBV24-1"
}